{
  "gene": "UniProtKB:O00562",
  "term_id": "GO:0008525",
  "term_label": "phosphatidylcholine transporter activity",
  "gene_name": "Membrane-associated phosphatidylinositol transfer protein 1",
  "gene_symbol": "PITPNM1"
}